regulation of angiotensin levels in blood [GO:0002002] (biological process) Relationships: is a type of regulation of hormone levels [GO:0010817]; is part of GO:0001991 Also known as: regulation of blood angiotensin level, control of angiotensin levels in blood, control of blood angiotensin level Definition: The process that modulates the level of any of the various angiotensinogen proteolytic products in the blood. This occurs by the proteolytic cleavage of angiotensinogen, and its proteolytic products, to create a variety of active peptide hormones, such as angiotensin I and angiotensin II, as well as through the removal of these peptides from the circulation. References: PMID:21951628 Sources: GOC:rl, Wikipedia:Angiotensin